{
  "term_label": "late endosome membrane",
  "gene_name": "HLA class II histocompatibility antigen, DRB1 beta chain",
  "gene": "UniProtKB:P01911",
  "term_id": "GO:0031902",
  "gene_symbol": "HLA-DRB1"
}